regulation of synapse pruning [GO:1905806] (biological process) Definition: Any process that modulates the frequency, rate or extent of synapse pruning. References: PMID:27779093 Sources: GOC:TermGenie, GO_REF:0000058 Also known as: regulation of synapse clearance, regulation of synapse disassembly, regulation of synapse elimination, regulation of synapse removal Relationships: is a type of regulation of synapse organization [GO:0050807]; regulates GO:0098883 Subtypes: negative regulation of synapse pruning [GO:1905807], positive regulation of synapse pruning [GO:1905808], GO:1905810